{
  "term_label": "nucleoplasm",
  "gene": "UniProtKB:O15151",
  "term_id": "GO:0005654",
  "gene_name": "Protein Mdm4",
  "gene_symbol": "MDM4"
}